nucleotide-excision repair, DNA damage recognition complex [GO:1990249] (cellular component) Definition: A protein complex that is capable of identifying lesions in DNA, such as pyrimidine-dimers, intrastrand cross-links, and bulky adducts. The wide range of substrate specificity suggests that the repair complex recognizes distortions in the DNA helix. It subsequently recruits a nucleotide-excision repair, preincision complex. References: PMID:22331906 Sources: GOC:bhm Relationships: is a type of protein-containing complex [GO:0032991] Subtypes: transcription-coupled nucleotide-excision repair, DNA damage recognition complex [GO:1990250]